regulation of epithelial cell proliferation involved in prostate gland development [GO:0060768] (biological process) Definition: Any process that modulates the rate, frequency or extent of epithelial cell proliferation that contributes to the progression of the prostate gland over time. Relationships: is a type of regulation of epithelial cell proliferation [GO:0050678]; regulates epithelial cell proliferation involved in prostate gland development [GO:0060767] Subtypes: positive regulation of epithelial cell proliferation involved in prostate gland development [GO:0060769], negative regulation of epithelial cell proliferation involved in prostate gland development [GO:0060770] Sources: GOC:dph